{
  "gene_symbol": "SLC2A14",
  "gene": "UniProtKB:Q8TDB8",
  "term_id": "GO:0046323",
  "gene_name": "Solute carrier family 2, facilitated glucose transporter member 14",
  "term_label": "D-glucose import"
}